{
  "term_id": "GO:0006357",
  "gene_name": "Zinc finger protein 14 homolog",
  "gene_symbol": "ZFP14",
  "term_label": "regulation of transcription by RNA polymerase II",
  "gene": "UniProtKB:Q9HCL3"
}